{
  "term_id": "GO:0007186",
  "term_label": "G protein-coupled receptor signaling pathway",
  "gene": "UniProtKB:Q9UBI6",
  "gene_symbol": "GNG12",
  "gene_name": "Guanine nucleotide-binding protein G(I)_G(S)_G(O) subunit gamma-12"
}